mitotic telomere maintenance via semi-conservative replication [GO:1902990] (biological process) Also known as: telomeric fork progression involved in mitotic cell cycle, telomeric replication fork progression involved in mitotic cell cycle, equal telomere replication involved in mitotic cell cycle Sources: GOC:TermGenie, GO_REF:0000060 Definition: Any telomere maintenance via semi-conservative replication that is involved in mitotic cell cycle. Relationships: is a type of GO:0032201; is a type of mitotic cell cycle process [GO:1903047]